cerebrospinal fluid circulation [GO:0090660] (biological process) Definition: The neurological system process driven by motile cilia on ependymal cells of the brain by which cerebrospinal fluid circulates from the sites of secretion to the sites of absorption. In ventricular cavities, the flow is unidirectional and rostrocaudal, in subarachnoid spaces, the flow is multi-directional. Also known as: CSF circulation, CSF flow, cerebrospinal fluid flow References: PMID:22100360, PMID:24229449 Sources: GOC:mgi_curators Relationships: is a type of epithelial cilium movement involved in extracellular fluid movement [GO:0003351]; is a type of nervous system process [GO:0050877]